{
  "term_id": "GO:0060339",
  "gene_name": "Small integral membrane protein 30",
  "gene": "UniProtKB:A4D0T7",
  "gene_symbol": "SMIM30",
  "term_label": "negative regulation of type I interferon-mediated signaling pathway"
}